{
  "term_id": "GO:0022008",
  "gene_name": "Fibroblast growth factor 22",
  "gene_symbol": "FGF22",
  "term_label": "neurogenesis",
  "gene": "UniProtKB:Q9HCT0"
}